{
  "term_id": "GO:0007507",
  "gene_symbol": "LDB3",
  "gene": "UniProtKB:O75112",
  "gene_name": "LIM domain-binding protein 3",
  "term_label": "heart development"
}